{
  "gene_name": "Bone sialoprotein 2",
  "gene_symbol": "IBSP",
  "term_id": "GO:0030282",
  "term_label": "bone mineralization",
  "gene": "UniProtKB:P21815"
}